{
  "gene_name": "Contactin-4",
  "term_label": "dendrite self-avoidance",
  "gene": "UniProtKB:Q8IWV2",
  "gene_symbol": "CNTN4",
  "term_id": "GO:0070593"
}